{
  "gene": "UniProtKB:P09132",
  "term_label": "signal recognition particle, endoplasmic reticulum targeting",
  "gene_name": "Signal recognition particle 19 kDa protein",
  "gene_symbol": "SRP19",
  "term_id": "GO:0005786"
}